{
  "gene_symbol": "NCR3",
  "gene": "UniProtKB:O14931",
  "term_id": "GO:0030101",
  "gene_name": "Natural cytotoxicity triggering receptor 3",
  "term_label": "natural killer cell activation"
}